{
  "gene_name": "EH domain-containing protein 4",
  "gene_symbol": "EHD4",
  "gene": "UniProtKB:Q9H223",
  "term_label": "endocytic vesicle",
  "term_id": "GO:0030139"
}